{
  "gene_symbol": "TMEM245",
  "gene": "UniProtKB:Q9H330",
  "term_id": "UNKNOWN:0001",
  "term_label": "Unknown molecular function",
  "gene_name": "Transmembrane protein 245"
}